death-inducing signaling complex [GO:0031264] (cellular component) Definition: A protein complex formed by the association of signaling proteins with a death receptor upon ligand binding. The complex includes procaspases and death domain-containing proteins in addition to the ligand-bound receptor, and may control the activation of caspases 8 and 10. Note: Gene products that may be annotated to this term include: 1) ligand-bound receptors such as FAS/CD95 (though care should be taken because FAS can also act as a non-apoptotic signal transducer); 2) signaling molecules such as FADD (FAS-associated protein with a death domain), cIAPs (cellular inhibitor of apoptosis proteins), c-FLIPs and caspases 8 and 10. Subtypes: GO:0031265, TRAIL death-inducing signaling complex [GO:0031266] References: PMID:12628743, PMID:12655293, PMID:8521815 Sources: GOC:mtg_apoptosis Also known as: DISC, DISC protein complex, death receptor-induced signaling complex, death receptor-induced signalling complex, death-inducing signalling complex Relationships: is a type of GO:0098797